{
  "gene": "UniProtKB:Q7L2J0",
  "gene_symbol": "MEPCE",
  "gene_name": "7SK snRNA methylphosphate capping enzyme",
  "term_id": "UNKNOWN:0003",
  "term_label": "Unknown cellular component"
}